nuclear polyadenylation-dependent snRNA catabolic process [GO:0071037] (BP) Also known as: nuclear poly(A)-dependent snRNA catabolic process Definition: The chemical reactions and pathways occurring in the nucleus and resulting in the breakdown of a small nuclear RNA (snRNA) molecule, initiated by the enzymatic addition of a sequence of adenylyl residues (polyadenylation) at the 3' end the target snRNA. Sources: GOC:dgf, GOC:krc Relationships: is a type of snRNA catabolic process [GO:0016076]; is a type of GO:0071027